CTP biosynthetic process [GO:0006241] (biological process) Sources: ISBN:0198506732 Definition: The chemical reactions and pathways resulting in the formation of CTP, cytidine 5'-triphosphate. Also known as: CTP anabolism, CTP biosynthesis, CTP formation, CTP synthesis Subtypes: 'de novo' CTP biosynthetic process [GO:0044210], CTP salvage [GO:0044211] Relationships: is a type of pyrimidine ribonucleoside triphosphate biosynthetic process [GO:0009209]; is a type of pyrimidine ribonucleotide biosynthetic process [GO:0009220]; is a type of CTP metabolic process [GO:0046036]